{
  "gene": "UniProtKB:Q93096",
  "gene_symbol": "PTP4A1",
  "term_label": "positive regulation of cell migration",
  "gene_name": "Protein tyrosine phosphatase type IVA 1",
  "term_id": "GO:0030335"
}